deoxynucleoside phosphate kinase activity, dTTP as phosphate donor [GO:0106368] (molecular function) Definition: Catalysis of the reaction: a 2'-deoxyribonucleoside 5'-phosphate + dTTP = a 2'-deoxyribonucleoside 5'-diphosphate + dTDP. References: PMID:20497505 Sources: RHEA:62132 Relationships: is a type of phosphotransferase activity, phosphate group as acceptor [GO:0016776]; is a type of nucleobase-containing compound kinase activity [GO:0019205]